{
  "gene_symbol": "A0A804HID5",
  "gene_name": "Uncharacterized protein",
  "term_label": "Unknown molecular function",
  "gene": "UniProtKB:A0A804HID5",
  "term_id": "UNKNOWN:0001"
}